{
  "gene": "UniProtKB:Q9NYW8",
  "gene_symbol": "RBAK",
  "gene_name": "RB-associated KRAB zinc finger protein",
  "term_id": "UNKNOWN:0003",
  "term_label": "Unknown cellular component"
}